{
  "gene_symbol": "PDE6A",
  "term_label": "negative regulation of cAMP/PKA signal transduction",
  "term_id": "GO:0141162",
  "gene": "UniProtKB:P16499",
  "gene_name": "Rod cGMP-specific 3',5'-cyclic phosphodiesterase subunit alpha"
}